{
  "gene_symbol": "PGBD1",
  "term_label": "sequence-specific DNA binding",
  "gene_name": "PiggyBac transposable element-derived protein 1",
  "gene": "UniProtKB:Q96JS3",
  "term_id": "GO:0043565"
}